{
  "gene_symbol": "SLC9A2",
  "term_id": "GO:0071805",
  "gene_name": "Sodium_hydrogen exchanger 2",
  "gene": "UniProtKB:Q9UBY0",
  "term_label": "potassium ion transmembrane transport"
}